{
  "gene_name": "Nuclear factor 1 A-type",
  "gene_symbol": "NFIA",
  "term_label": "RNA polymerase II cis-regulatory region sequence-specific DNA binding",
  "term_id": "GO:0000978",
  "gene": "UniProtKB:Q12857"
}